{
  "gene_name": "InaD-like protein",
  "term_label": "Unknown molecular function",
  "gene_symbol": "PATJ",
  "term_id": "UNKNOWN:0001",
  "gene": "UniProtKB:Q8NI35"
}